{
  "gene_symbol": "CT47A12",
  "gene_name": "Cancer_testis antigen 47A",
  "term_id": "UNKNOWN:0003",
  "gene": "UniProtKB:Q5JQC4",
  "term_label": "Unknown cellular component"
}